{
  "gene_symbol": "PTPN5",
  "term_id": "GO:0004725",
  "term_label": "protein tyrosine phosphatase activity",
  "gene": "UniProtKB:P54829",
  "gene_name": "Tyrosine-protein phosphatase non-receptor type 5"
}